syncytium formation by mitosis without cytokinesis [GO:0000769] (biological process) Definition: The formation of a syncytium, a mass of cytoplasm containing several nuclei enclosed within a single plasma membrane, by one or more rounds of nuclear division without cytokinesis. Also known as: syncytium formation by mitosis without cell division Sources: GOC:mah, GOC:tb Relationships: is a type of syncytium formation [GO:0006949]; has part cell cycle comprising mitosis without cytokinesis [GO:0033301]